podocyte cell fate commitment [GO:0072149] (biological process) Also known as: glomerular visceral epithelial cell fate commitment Definition: The process in which the developmental fate of a cell becomes restricted such that it will develop into a glomerular visceral epithelial cell. A glomerular visceral epithelial cell is a specialized epithelial cell that contains 'feet' that interdigitate with the 'feet' of other glomerular epithelial cells. Sources: GOC:mtg_kidney_jan10 Subtypes: mesonephric podocyte cell fate commitment [GO:0061258], GO:0072250 Relationships: is a type of epithelial cell fate commitment [GO:0072148]; is a type of GO:0072314; is part of GO:0072112